{
  "term_label": "Unknown cellular component",
  "term_id": "UNKNOWN:0003",
  "gene_name": "Putative uncharacterized protein CCDC28A-AS1",
  "gene": "UniProtKB:A0A096LPI5",
  "gene_symbol": "CCDC28A-AS1"
}